symbiont-mediated suppression of host translation initiation [GO:0039606] (biological process) Also known as: suppression by virus of host translation initiation Sources: GOC:bf Relationships: is a type of GO:0039656 Definition: A process in which a symbiont inhibits or disrupts translation initiation in its host. The host is defined as the larger of the organisms involved in a symbiotic interaction.